{
  "gene_name": "Cyclin-P",
  "term_id": "GO:0005737",
  "term_label": "cytoplasm",
  "gene": "UniProtKB:Q9H8S5",
  "gene_symbol": "CCNP"
}